filamin binding [GO:0031005] (molecular function) Definition: Binding to a filamin, any member of a family of high molecular mass cytoskeletal proteins that crosslink actin filaments to form networks and stress fibers. Filamins contain an amino-terminal alpha-actinin-like actin binding domain, which is followed by a rod-domain composed of 4 to 24 100-residue repetitive segments including a carboxy-terminal dimerization domain. References: PMID:11336782 Sources: GOC:mah Also known as: filamin C binding, filamin-B binding, ABP-278/276 binding, ABP-280 binding, ABPL binding, alpha-filamin binding, beta-filamin binding, filamin A binding, filamin B binding, filamin-1 binding, filamin-2 binding, filamin-3 binding, filamin-A binding, filamin-C binding, gamma-filamin binding Relationships: is a type of cytoskeletal protein binding [GO:0008092]